regulation of microglial cell mediated cytotoxicity [GO:1904149] (biological process) Subtypes: negative regulation of microglial cell mediated cytotoxicity [GO:1904150], GO:1904151 References: PMID:19100238 Sources: GOC:BHF, GOC:TermGenie, GOC:nc, GO_REF:0000058 Relationships: is a type of regulation of leukocyte mediated cytotoxicity [GO:0001910]; is a type of regulation of myeloid leukocyte mediated immunity [GO:0002886]; regulates microglial cell mediated cytotoxicity [GO:0090634] Definition: Any process that modulates the frequency, rate or extent of microglial cell mediated cytotoxicity.